negative gravitaxis [GO:0048060] (biological process) Also known as: negative geotactic behavior, negative geotactic behaviour, negative gravitactic behavior, negative gravitactic behaviour, negative taxis in response to gravity, negative taxis in response to gravitytaxis in response to gravitational stimulus Relationships: is a type of gravitaxis [GO:0042332] Sources: GOC:jid Definition: The directed movement of a motile cell or organism away from the source of gravity.